negative regulation of cell-cell adhesion mediated by integrin [GO:0033633] (biological process) Also known as: negative regulation of cell-cell adhesion mediated by integrin complex Definition: Any process that stops, prevents, or reduces the frequency, rate, or extent of cell-cell adhesion mediated by integrin. Relationships: is a type of negative regulation of cell-cell adhesion [GO:0022408]; is a type of negative regulation of cell adhesion mediated by integrin [GO:0033629]; is a type of regulation of cell-cell adhesion mediated by integrin [GO:0033632]; negatively regulates GO:0033631 Sources: GOC:add